{
  "gene_symbol": "CLEC1B",
  "term_id": "GO:0005886",
  "gene": "UniProtKB:Q9P126",
  "term_label": "plasma membrane",
  "gene_name": "C-type lectin domain family 1 member B"
}